{
  "term_id": "GO:0005587",
  "term_label": "collagen type IV trimer",
  "gene": "UniProtKB:P02462",
  "gene_name": "Collagen alpha-1(IV) chain",
  "gene_symbol": "COL4A1"
}